prebend segment development [GO:0072066] (biological process) Relationships: is a type of tube development [GO:0035295]; is part of descending thin limb development [GO:0072022] Sources: GOC:mtg_kidney_jan10 Subtypes: metanephric prebend segment development [GO:0072228] Definition: The process whose specific outcome is the progression of the prebend segment over time, from its formation to the mature structure. The prebend segment is a part of the descending thin limb that lies before the bend and exhibits permeabilities characteristic of the ascending limb, especially negligible water permeability.